histidine-tRNA ligase activity [GO:0004821] (molecular function) Definition: Catalysis of the reaction: ATP + L-histidine + tRNA(His) = AMP + diphosphate + L-histidyl-tRNA(His). Sources: EC:6.1.1.21 Also known as: histidyl-tRNA synthetase activity, L-histidine:tRNAHis ligase (AMP-forming), histidine translase activity, histidyl-transfer ribonucleate synthetase activity Relationships: is a type of aminoacyl-tRNA ligase activity [GO:0004812]